{
  "term_id": "UNKNOWN:0003",
  "gene": "UniProtKB:Q9P2D6",
  "gene_name": "Protein FAM135A",
  "gene_symbol": "FAM135A",
  "term_label": "Unknown cellular component"
}